{
  "gene": "UniProtKB:Q9UK23",
  "term_label": "Unknown molecular function",
  "gene_name": "N-acetylglucosamine-1-phosphodiester alpha-N-acetylglucosaminidase",
  "gene_symbol": "NAGPA",
  "term_id": "UNKNOWN:0001"
}